SeqA-DNA complex [GO:1990097] (cellular component) Also known as: SeqA-dsDNA complex, SeqA-hemimethylated DNA complex, SeqA-hemimethylation dsDNA complex References: PMID:12379844, PMID:15933720, PMID:23149570 Sources: GOC:bhm Relationships: is a type of protein-DNA complex [GO:0032993] Definition: A protein-DNA complex that contains an oligomer of SeqA bound to GATC sites in methylated or newly-synthesized, hemi-methylated double-stranded DNA, with preference for the latter. Binding of SeqA to hemimethylated DNA sequesters oriC, prevents re-methylation of DNA by Dam and in turn stops premature re-initiation of replication during one replication cycle.